{
  "term_id": "GO:0031491",
  "gene_symbol": "GLYR1",
  "term_label": "nucleosome binding",
  "gene": "UniProtKB:Q49A26",
  "gene_name": "Cytokine-like nuclear factor N-PAC"
}